{
  "term_label": "BRCA1-BARD1 complex",
  "term_id": "GO:0031436",
  "gene_symbol": "BARD1",
  "gene": "UniProtKB:Q99728",
  "gene_name": "BRCA1-associated RING domain protein 1"
}